{
  "gene_name": "Kinase suppressor of Ras 1",
  "gene_symbol": "KSR1",
  "term_id": "GO:0005737",
  "gene": "UniProtKB:Q8IVT5",
  "term_label": "cytoplasm"
}